{
  "gene": "UniProtKB:Q8N6N3",
  "gene_name": "UPF0690 protein C1orf52",
  "term_id": "UNKNOWN:0001",
  "term_label": "Unknown molecular function",
  "gene_symbol": "C1orf52"
}